{
  "gene_symbol": "TAS2R46",
  "term_label": "detection of chemical stimulus involved in sensory perception of bitter taste",
  "term_id": "GO:0001580",
  "gene_name": "Taste receptor type 2 member 46",
  "gene": "UniProtKB:P59540"
}